{
  "term_label": "endoplasmic reticulum organization",
  "gene_name": "Atlastin-1",
  "gene_symbol": "ATL1",
  "term_id": "GO:0007029",
  "gene": "UniProtKB:Q8WXF7"
}